tRNA nucleoside ribose methylation [GO:0002128] (biological process) Relationships: is_a GO:0030488 Sources: GOC:hjd, ISBN:155581073X Subtypes: wobble position ribose methylation [GO:0002130], tRNA guanine ribose methylation [GO:0002938] Definition: The process that results in the modification of the sugar of a nucleoside in tRNA at the 2'O position.